{
  "gene": "UniProtKB:O75340",
  "term_label": "Unknown cellular component",
  "term_id": "UNKNOWN:0003",
  "gene_name": "Programmed cell death protein 6",
  "gene_symbol": "PDCD6"
}